(2R)-hydroxyphenylpyruvate reductase [NAD(P)H] activity [GO:0047995] (molecular function) Also known as: 4-hydroxyphenyllactate:NAD+ oxidoreductase activity, HPRP Sources: EC:1.1.1.237 Definition: Catalysis of the reaction: (2R)-2-hydroxy-3-(4-hydroxyphenyl)propanoate + NAD(P)+ = 3-(4-hydroxyphenyl)pyruvate + NAD(P)H + H+. Relationships: is a type of (2R)-2-hydroxyacid dehydrogenase (NAD+) activity [GO:0140175]